{
  "gene": "UniProtKB:P26038",
  "gene_symbol": "MSN",
  "gene_name": "Moesin",
  "term_label": "regulation of cell shape",
  "term_id": "GO:0008360"
}